{
  "gene_name": "Pantothenate kinase 2, mitochondrial",
  "gene_symbol": "PANK2",
  "gene": "UniProtKB:Q9BZ23",
  "term_id": "GO:0005634",
  "term_label": "nucleus"
}